{
  "gene": "UniProtKB:Q5EBM0",
  "gene_symbol": "CMPK2",
  "gene_name": "UMP-CMP kinase 2, mitochondrial",
  "term_id": "GO:0005737",
  "term_label": "cytoplasm"
}